stereocilium coat [GO:0120234] (CC) Relationships: is a type of glycocalyx [GO:0030112]; is part of GO:0032420 References: PMID:31444330, PMID:3583936 Sources: GOC:krc, ISBN:9781461268918 Also known as: auditory hair cell glycocalyx, stereocilium glycocalyx Definition: A glycocalyx on the the endolymphatic surface of a cochlear hair cell that coats the external surface of each stereocilium and maintains a small distance between adjacent stereocilia in the bundle.